{
  "term_id": "GO:0003712",
  "gene": "UniProtKB:P51825",
  "gene_symbol": "AFF1",
  "gene_name": "AF4_FMR2 family member 1",
  "term_label": "transcription coregulator activity"
}